{
  "term_id": "GO:0000978",
  "term_label": "RNA polymerase II cis-regulatory region sequence-specific DNA binding",
  "gene_name": "Nuclear transcription factor Y subunit gamma",
  "gene": "UniProtKB:Q13952",
  "gene_symbol": "NFYC"
}